anterior mesonephric tubule development [GO:0072165] (biological process) Sources: GOC:mtg_kidney_jan10 Definition: The progression of the anterior mesonephric tubule over time, from its initial formation to the mature structure. The anterior mesonephric tubule is an epithelial tube that is part of the mesonephros. Relationships: is a type of mesonephric tubule development [GO:0072164]